{
  "gene": "UniProtKB:Q49SQ1",
  "gene_name": "Probable G-protein coupled receptor 33",
  "term_label": "plasma membrane",
  "term_id": "GO:0005886",
  "gene_symbol": "GPR33"
}